cyclic nucleotide biosynthetic process [GO:0009190] (biological process) Definition: The chemical reactions and pathways resulting in the formation of a cyclic nucleotide, a nucleotide in which the phosphate group is in diester linkage to two positions on the sugar residue. Subtypes: cAMP biosynthetic process [GO:0006171], cGMP biosynthetic process [GO:0006182] Sources: GOC:go_curators, ISBN:0198506732 Also known as: cyclic nucleotide anabolism, cyclic nucleotide biosynthesis, cyclic nucleotide formation, cyclic nucleotide synthesis Relationships: is a type of GO:0009165; is a type of GO:0009187